regulation of plant-type hypersensitive response [GO:0010363] (biological process) Definition: Any endogenous process that modulates the frequency, rate or extent of the plant hypersensitive response. References: PMID:16255244 Subtypes: GO:0034051, positive regulation of plant-type hypersensitive response [GO:0034052] Note: Note that term is to be used to annotate gene products in the plant. To annotate genes in a symbiont, consider the biological process term 'modulation by symbiont of host programmed cell death ; GO:0052040'. Also known as: regulation of HR, regulation of HR-PCD, regulation of plant hypersensitive response Relationships: is a type of GO:0043067; is_a GO:0045088; is a type of GO:0080135; regulates plant-type hypersensitive response [GO:0009626]